{
  "gene_symbol": "IL6ST",
  "term_label": "receptor complex",
  "gene": "UniProtKB:P40189",
  "term_id": "GO:0043235",
  "gene_name": "Interleukin-6 receptor subunit beta"
}